protein catabolic process at synapse [GO:0140246] (biological process) Note: Note that this term was created for the SynGO project, and will be obsoleted when the SynGO annotations are made in Noctua. Subtypes: protein catabolic process, modulating synaptic transmission [GO:0099546], GO:0140247, protein catabolic process at postsynapse [GO:0140249] References: PMID:17062563 Relationships: is a type of protein catabolic process [GO:0030163]; BFO_0000066 synapse [GO:0045202] Definition: The chemical reactions and pathways resulting in the breakdown of a protein at a synapse.